{
  "term_id": "GO:0045954",
  "gene": "UniProtKB:O14931",
  "term_label": "positive regulation of natural killer cell mediated cytotoxicity",
  "gene_symbol": "NCR3",
  "gene_name": "Natural cytotoxicity triggering receptor 3"
}